{
  "gene_symbol": "PFKL",
  "gene_name": "ATP-dependent 6-phosphofructokinase, liver type",
  "term_id": "GO:0061621",
  "gene": "UniProtKB:P17858",
  "term_label": "canonical glycolysis"
}